{
  "term_id": "GO:0050778",
  "gene_name": "HLA class II histocompatibility antigen, DP beta 1 chain",
  "gene": "UniProtKB:P04440",
  "term_label": "positive regulation of immune response",
  "gene_symbol": "HLA-DPB1"
}